{
  "term_label": "Unknown biological process",
  "gene_symbol": "BCR",
  "gene_name": "Breakpoint cluster region protein",
  "gene": "UniProtKB:P11274",
  "term_id": "UNKNOWN:0002"
}